{
  "term_label": "negative regulation of thymocyte apoptotic process",
  "term_id": "GO:0070244",
  "gene_name": "Pre T-cell antigen receptor alpha",
  "gene": "UniProtKB:Q6ISU1",
  "gene_symbol": "PTCRA"
}